thyroxine 5'-deiodinase activity [GO:0004800] (molecular function) Relationships: is a type of oxidoreductase activity, acting on X-H and Y-H to form an X-Y bond [GO:0046992] Also known as: thyroxine deiodinase activity, outer ring-deiodinating pathway, thyroxine 5' deiodinase activity, type I iodothyronine deiodinase activity, type II iodothyronine deiodinase activity, L-thyroxine iodohydrolase (reducing) activity, acceptor:3,5,3'-triiodo-L-thyronine oxidoreductase (iodinating), diiodothyronine 5'-deiodinase activity, iodothyronine 5'-deiodinase activity, iodothyronine outer ring monodeiodinase activity Definition: Catalysis of the reaction: 3,3',5-triiodo-L-thyronine + iodide + acceptor + H+ = L-thyroxine + acceptor-H2. Sources: RHEA:19745